cerebellar molecular layer formation [GO:0021688] (biological process) Definition: The process that gives rise to the cerebellar molecular layer. This process pertains to the initial formation of a structure from unspecified parts. The molecular layer is the outermost layer of the cerebellar cortex. It contains the parallel fibers of the granule cells, interneurons such as stellate and basket cells, and the dendrites of the underlying Purkinje cells. Sources: GOC:cls, GOC:dgh, GOC:dph, GOC:jid, GO_REF:0000021 Relationships: is a type of anatomical structure formation involved in morphogenesis [GO:0048646]; is part of GO:0021687; is part of cerebellar cortex formation [GO:0021697]